{
  "term_id": "GO:0070053",
  "gene_name": "Leukocyte surface antigen CD47",
  "term_label": "thrombospondin receptor activity",
  "gene": "UniProtKB:Q08722",
  "gene_symbol": "CD47"
}